{
  "term_label": "nucleus",
  "gene": "UniProtKB:Q96J87",
  "gene_symbol": "CELF6",
  "term_id": "GO:0005634",
  "gene_name": "CUGBP Elav-like family member 6"
}